{
  "term_id": "GO:0000278",
  "gene_name": "Spindle and kinetochore-associated protein 1",
  "gene_symbol": "SKA1",
  "gene": "UniProtKB:Q96BD8",
  "term_label": "mitotic cell cycle"
}